regulation of cytoplasmic translation in response to stress [GO:1990497] (biological process) Relationships: is a type of regulation of translation in response to stress [GO:0043555]; is_a GO:2000765 Subtypes: regulation of cytoplasmic translational initiation in response to stress [GO:1990611] Definition: Modulation of the frequency, rate or extent of cytoplasmic translation as a result of a stimulus indicating the organism is under stress. The stress is usually, but not necessarily, exogenous (e.g. temperature, humidity, ionizing radiation). References: PMID:16278445 Sources: GOC:vw